{
  "gene_symbol": "LRCH2",
  "gene_name": "Leucine-rich repeat and calponin homology domain-containing protein 2",
  "gene": "UniProtKB:Q5VUJ6",
  "term_id": "UNKNOWN:0003",
  "term_label": "Unknown cellular component"
}